{
  "term_id": "UNKNOWN:0002",
  "gene": "UniProtKB:Q9NX78",
  "gene_symbol": "TMEM260",
  "gene_name": "Transmembrane protein 260",
  "term_label": "Unknown biological process"
}